rhodopsin biosynthetic process [GO:0016063] (biological process) Sources: ISBN:0198506732 Also known as: rhodopsin anabolism, rhodopsin biosynthesis, rhodopsin formation, rhodopsin synthesis Relationships: is a type of eye pigment biosynthetic process [GO:0006726]; is a type of macromolecule biosynthetic process [GO:0009059]; is_a rhodopsin metabolic process [GO:0046154] Definition: The chemical reactions and pathways resulting in the formation of rhodopsin, a brilliant purplish-red, light-sensitive visual pigment found in the rod cells of the retinas.